{
  "gene_name": "Bone morphogenetic protein 15",
  "gene_symbol": "BMP15",
  "term_label": "extracellular space",
  "gene": "UniProtKB:O95972",
  "term_id": "GO:0005615"
}